COPI-coated vesicle membrane [GO:0030663] (cellular component) Also known as: COPI coated vesicle membrane Subtypes: Golgi to ER transport vesicle membrane [GO:0012508], inter-Golgi transport vesicle membrane [GO:0012509] Relationships: is a type of GO:0030660; is_a coated vesicle membrane [GO:0030662]; is part of GO:0030137 Definition: The lipid bilayer surrounding a COPI-coated vesicle. Sources: GOC:mah